{
  "gene": "UniProtKB:A6NCN8",
  "gene_name": "Testis-expressed protein 52",
  "term_id": "UNKNOWN:0002",
  "term_label": "Unknown biological process",
  "gene_symbol": "TEX52"
}